toluene oxidation via 3-hydroxytoluene [GO:0019602] (biological process) Definition: The degradation of toluene to form pyruvate and acetaldehyde; the first step in the pathway is the oxidation of toluene to form 3-hydroxytoluene (m-cresol). Sources: MetaCyc:TOLUENE-DEG-3-OH-PWY Relationships: is_a toluene oxidation [GO:0019600]